negative regulation of compound eye pigmentation [GO:0048077] (biological process) Sources: GOC:jid Relationships: is a type of negative regulation of eye pigmentation [GO:0048074]; is a type of GO:0048076; negatively regulates compound eye pigmentation [GO:0048072] Definition: Any process that stops, prevents, or reduces the frequency, rate or extent of establishment of a pattern of pigment in the compound eye. Also known as: down regulation of eye pigmentation, down-regulation of eye pigmentation, downregulation of eye pigmentation, inhibition of eye pigmentation, negative regulation of eye pigmentation